{
  "gene_symbol": "AHNAK",
  "term_label": "Unknown molecular function",
  "term_id": "UNKNOWN:0001",
  "gene": "UniProtKB:Q09666",
  "gene_name": "Neuroblast differentiation-associated protein AHNAK"
}